{
  "term_id": "GO:0016309",
  "gene_symbol": "PIP4K2B",
  "term_label": "1-phosphatidylinositol-5-phosphate 4-kinase activity",
  "gene": "UniProtKB:P78356",
  "gene_name": "Phosphatidylinositol 5-phosphate 4-kinase type-2 beta"
}